long descending thin limb bend development [GO:0072065] (BP) Definition: The process whose specific outcome is the progression of the long descending thin limb bend over time, from its formation to the mature structure. The long descending thin limb bend is a part of the descending thin limb of a long nephron that lies beyond the prebend segment. Sources: GOC:mtg_kidney_jan10 Relationships: is a type of tube development [GO:0035295]; is part of long descending thin limb development [GO:0072064] Subtypes: metanephric long descending thin limb bend development [GO:0072226]